{
  "term_label": "Unknown cellular component",
  "gene": "UniProtKB:A6NJ69",
  "gene_name": "IgA-inducing protein homolog",
  "gene_symbol": "IGIP",
  "term_id": "UNKNOWN:0003"
}